{
  "term_id": "GO:0050839",
  "term_label": "cell adhesion molecule binding",
  "gene_symbol": "TJP3",
  "gene": "UniProtKB:O95049",
  "gene_name": "Tight junction protein ZO-3"
}